complement component C1q complex binding [GO:0001849] (molecular function) Definition: Binding to a C1q complex, a component of the classical complement cascade. Relationships: is a type of opsonin binding [GO:0001846]; is a type of GO:0001848; is a type of protein-containing complex binding [GO:0044877] Sources: GOC:add, ISBN:0781735149